{
  "term_id": "UNKNOWN:0001",
  "term_label": "Unknown molecular function",
  "gene_name": "Armadillo repeat-containing protein 3",
  "gene_symbol": "ARMC3",
  "gene": "UniProtKB:Q5W041"
}